{
  "gene": "UniProtKB:Q8NGB8",
  "gene_symbol": "OR4F15",
  "term_id": "UNKNOWN:0003",
  "gene_name": "Olfactory receptor 4F15",
  "term_label": "Unknown cellular component"
}